{
  "term_id": "GO:0004971",
  "term_label": "AMPA glutamate receptor activity",
  "gene_name": "Glutamate receptor 4",
  "gene_symbol": "GRIA4",
  "gene": "UniProtKB:P48058"
}